{
  "term_label": "synaptic vesicle fusion to presynaptic active zone membrane",
  "gene_name": "Syntaxin-11",
  "gene": "UniProtKB:O75558",
  "gene_symbol": "STX11",
  "term_id": "GO:0031629"
}